{
  "gene": "UniProtKB:Q2TBA0",
  "term_label": "skeletal muscle fiber development",
  "gene_name": "Kelch-like protein 40",
  "term_id": "GO:0048741",
  "gene_symbol": "KLHL40"
}